{
  "gene_symbol": "SQSTM1",
  "gene_name": "Sequestosome-1",
  "gene": "UniProtKB:Q13501",
  "term_id": "GO:0035973",
  "term_label": "aggrephagy"
}